{
  "gene": "UniProtKB:Q9NRJ3",
  "gene_symbol": "CCL28",
  "term_id": "GO:0061844",
  "term_label": "antimicrobial humoral immune response mediated by antimicrobial peptide",
  "gene_name": "C-C motif chemokine 28"
}